{
  "gene_symbol": "TRAV35",
  "term_id": "UNKNOWN:0001",
  "gene_name": "T cell receptor alpha variable 35",
  "gene": "UniProtKB:P0DPF4",
  "term_label": "Unknown molecular function"
}